{
  "gene_name": "Telomere repeats-binding bouquet formation protein 2",
  "term_label": "nuclear inner membrane",
  "gene_symbol": "TERB2",
  "gene": "UniProtKB:Q8NHR7",
  "term_id": "GO:0005637"
}